{
  "term_label": "lysosomal membrane",
  "gene_name": "E3 ubiquitin-protein ligase TRIM23",
  "gene": "UniProtKB:P36406",
  "gene_symbol": "TRIM23",
  "term_id": "GO:0005765"
}